{
  "gene_symbol": "TRPC1",
  "term_label": "store-operated calcium channel activity",
  "term_id": "GO:0015279",
  "gene": "UniProtKB:P48995",
  "gene_name": "Short transient receptor potential channel 1"
}